long-chain fatty acid transmembrane transporter activity [GO:0005324] (molecular function) Relationships: is a type of fatty acid transmembrane transporter activity [GO:0015245]; is part of long-chain fatty acid transport [GO:0015909] Sources: ISBN:0198506732 Definition: Enables the transfer of a long-chain fatty acid from one side of a membrane to the other. A long-chain fatty acid has an aliphatic tail containing 13 to 22 carbons. Also known as: long-chain fatty acid transporter activity Subtypes: GO:0015483, oleate transmembrane transporter activity [GO:1901480], arachidonate transmembrane transporter activity [GO:1903962] Note: While there is not universal consensus on the lengths of short-, medium-, long- and very-long-chain fatty acids, the GO uses the definitions in ChEBI (see CHEBI:26666, CHEBI:59554, CHEBI:15904 and CHEBI:27283).